{
  "gene": "UniProtKB:A0A0C4DH43",
  "term_id": "GO:0003823",
  "gene_name": "Immunoglobulin heavy variable 2-70D",
  "term_label": "antigen binding",
  "gene_symbol": "IGHV2-70D"
}